{
  "term_id": "GO:0008037",
  "term_label": "cell recognition",
  "gene": "UniProtKB:O95727",
  "gene_name": "Cytotoxic and regulatory T-cell molecule",
  "gene_symbol": "CRTAM"
}